{
  "term_label": "antifungal innate immune response",
  "gene_symbol": "CLEC4C",
  "gene": "UniProtKB:Q8WTT0",
  "gene_name": "C-type lectin domain family 4 member C",
  "term_id": "GO:0061760"
}